{
  "term_id": "UNKNOWN:0001",
  "term_label": "Unknown molecular function",
  "gene_symbol": "UQCRC1",
  "gene": "UniProtKB:P31930",
  "gene_name": "Cytochrome b-c1 complex subunit 1, mitochondrial"
}